{
  "term_id": "UNKNOWN:0003",
  "gene_symbol": "GGTLC1",
  "term_label": "Unknown cellular component",
  "gene_name": "Glutathione hydrolase light chain 1",
  "gene": "UniProtKB:Q9BX51"
}